regulation of receptor-mediated virion attachment to host cell [GO:1902734] (biological process) References: PMID:18385238 Sources: GOC:TermGenie, GOC:als, GO_REF:0000058 Definition: Any process that modulates the frequency, rate or extent of receptor-mediated virion attachment to host cell. Also known as: regulation of virion attachment, binding of host cell surface receptor Subtypes: GO:1902735, GO:1902736 Relationships: is a type of regulation of biological process involved in symbiotic interaction [GO:0043903]; is_a regulation of viral life cycle [GO:1903900]; regulates GO:0046813